{
  "term_label": "chemokine activity",
  "gene_symbol": "CCL25",
  "term_id": "GO:0008009",
  "gene_name": "C-C motif chemokine 25",
  "gene": "UniProtKB:O15444"
}